regulation of nerve growth factor production [GO:0032903] (BP) Definition: Any process that modulates the frequency, rate, or extent of production of nerve growth factor (NGF). Sources: GOC:mah Also known as: regulation of NGF production, regulation of beta-nerve growth factor production Relationships: is a type of regulation of neurotrophin production [GO:0032899]; regulates nerve growth factor production [GO:0032902] Subtypes: negative regulation of nerve growth factor production [GO:0032904]